{
  "gene_name": "Deoxyribonuclease-2-beta",
  "term_id": "GO:0004531",
  "term_label": "deoxyribonuclease II activity",
  "gene_symbol": "DNASE2B",
  "gene": "UniProtKB:Q8WZ79"
}